{
  "term_label": "negative regulation of actin filament polymerization",
  "gene_symbol": "SSH1",
  "gene": "UniProtKB:Q8WYL5",
  "term_id": "GO:0030837",
  "gene_name": "Protein phosphatase Slingshot homolog 1"
}